homogalacturonan catabolic process [GO:0033393] (biological process) Definition: The chemical reactions and pathways resulting in the breakdown of homogalacturonan, a pectidic polymer, characterized by a backbone of 1,4-linked alpha-D-GalpA residues that can be methyl-esterified at C-6 and carry acetyl groups on O-2 and O-3. Sources: GOC:mah Also known as: homogalacturonan breakdown, homogalacturonan catabolism, homogalacturonan degradation Relationships: is a type of polysaccharide catabolic process [GO:0000272]; is a type of homogalacturonan metabolic process [GO:0010394]